{
  "gene_symbol": "FUS",
  "term_label": "RNA binding",
  "gene": "UniProtKB:P35637",
  "gene_name": "RNA-binding protein FUS",
  "term_id": "GO:0003723"
}